{
  "gene_symbol": "STAT6",
  "term_label": "cytoplasm",
  "gene_name": "Signal transducer and activator of transcription 6",
  "term_id": "GO:0005737",
  "gene": "UniProtKB:P42226"
}